{
  "gene_symbol": "EVC2",
  "term_id": "UNKNOWN:0001",
  "gene_name": "Limbin",
  "term_label": "Unknown molecular function",
  "gene": "UniProtKB:Q86UK5"
}